{
  "term_label": "extracellular matrix",
  "gene": "UniProtKB:Q8IZC6",
  "gene_symbol": "COL27A1",
  "gene_name": "Collagen alpha-1(XXVII) chain",
  "term_id": "GO:0031012"
}